{
  "term_id": "GO:0047952",
  "gene_symbol": "GPD1",
  "gene_name": "Glycerol-3-phosphate dehydrogenase [NAD(+)], cytoplasmic",
  "term_label": "glycerol-3-phosphate dehydrogenase [NAD(P)+] activity",
  "gene": "UniProtKB:P21695"
}